{
  "term_id": "UNKNOWN:0002",
  "gene": "UniProtKB:O95154",
  "term_label": "Unknown biological process",
  "gene_symbol": "AKR7A3",
  "gene_name": "Aflatoxin B1 aldehyde reductase member 3"
}